{
  "term_label": "zinc ion transmembrane transport",
  "gene_name": "Zinc transporter SLC39A7",
  "term_id": "GO:0071577",
  "gene": "UniProtKB:Q92504",
  "gene_symbol": "SLC39A7"
}